response to tetrahydrofolate [GO:1904481] (biological process) Relationships: is a type of GO:1901698; is a type of GO:1901700 References: PMID:24698160 Sources: GOC:BHF, GOC:TermGenie, GOC:hal, GO_REF:0000071 Definition: Any process that results in a change in state or activity of a cell or an organism (in terms of movement, secretion, enzyme production, gene expression, etc.) as a result of a tetrahydrofolate stimulus. Subtypes: cellular response to tetrahydrofolate [GO:1904482]